oxidoreductase activity, acting on the CH-CH group of donors, oxygen as acceptor [GO:0016634] (molecular function) Definition: Catalysis of an oxidation-reduction (redox) reaction in which a CH-CH group acts as a hydrogen or electron donor and reduces oxygen. Relationships: is a type of oxidoreductase activity, acting on the CH-CH group of donors [GO:0016627] Subtypes: acyl-CoA oxidase activity [GO:0003997], coproporphyrinogen oxidase activity [GO:0004109], GO:0004729, pyrroloquinoline-quinone synthase activity [GO:0033732], bilirubin oxidase activity [GO:0047705], dihydrouracil oxidase activity [GO:0047857], L-galactonolactone oxidase activity [GO:0050024], tetrahydroberberine oxidase activity [GO:0050328], GO:0050541, GO:0050616, tryptophan alpha,beta-oxidase activity [GO:0050621] Sources: EC:1.3.3.-